biotin carboxyl carrier protein biosynthetic process [GO:0042966] (biological process) Definition: The chemical reactions and pathways resulting in the formation of the biotin carboxyl carrier protein, a subunit of acetyl-coenzyme A carboxylase. Also known as: BCCP biosynthesis, BCCP biosynthetic process, biotin carboxyl carrier protein anabolism, biotin carboxyl carrier protein biosynthesis, biotin carboxyl carrier protein formation, biotin carboxyl carrier protein synthesis Relationships: is a type of GO:0009059 References: PMID:8102363 Sources: GOC:go_curators